substrate localization to autophagosome [GO:0061753] (biological process) Relationships: is a type of establishment of localization in cell [GO:0051649]; is part of autophagosome assembly [GO:0000045] Definition: The localization process by which an autophagic substrate is delivered to a forming autophagosome. Also known as: substrate sequestration to autophagosome, substrate sequestration to phagophore References: PMID:23545414 Sources: GOC:PARL, GOC:dph, GOC:pad